{
  "gene": "UniProtKB:P42345",
  "term_label": "cytoplasm",
  "term_id": "GO:0005737",
  "gene_name": "Serine_threonine-protein kinase mTOR",
  "gene_symbol": "MTOR"
}